{
  "term_label": "structural molecule activity",
  "term_id": "GO:0005198",
  "gene_name": "Desmoplakin",
  "gene": "UniProtKB:P15924",
  "gene_symbol": "DSP"
}